{
  "term_label": "proteolysis",
  "gene_name": "Endoplasmic reticulum metallopeptidase 1",
  "gene_symbol": "ERMP1",
  "gene": "UniProtKB:Q7Z2K6",
  "term_id": "GO:0006508"
}